{
  "gene_name": "Lysophospholipase D GDPD1",
  "term_label": "N-acylethanolamine metabolic process",
  "gene_symbol": "GDPD1",
  "gene": "UniProtKB:Q8N9F7",
  "term_id": "GO:0070291"
}